regulation of iodide transport [GO:1904201] (biological process) Relationships: is a type of regulation of monoatomic anion transport [GO:0044070]; regulates iodide transport [GO:0015705] References: PMID:20392814 Sources: GOC:TermGenie, GO_REF:0000058 Definition: Any process that modulates the frequency, rate or extent of iodide transport. Subtypes: negative regulation of iodide transport [GO:1904202], positive regulation of iodide transport [GO:1904203], regulation of iodide transmembrane transport [GO:1904212]